{
  "term_id": "UNKNOWN:0002",
  "gene": "UniProtKB:P02812",
  "term_label": "Unknown biological process",
  "gene_symbol": "PRB2",
  "gene_name": "Basic salivary proline-rich protein 2"
}